{
  "term_label": "lipid oxidation",
  "gene": "UniProtKB:O75342",
  "gene_name": "Arachidonate 12-lipoxygenase, 12R-type",
  "term_id": "GO:0034440",
  "gene_symbol": "ALOX12B"
}